positive regulation of response to endoplasmic reticulum stress [GO:1905898] (BP) Also known as: positive regulation of ER stress response, positive regulation of cellular response to endoplasmic reticulum stress, positive regulation of response to ER stress, up regulation of ER stress response, up regulation of cellular response to endoplasmic reticulum stress, up regulation of response to ER stress, up regulation of response to endoplasmic reticulum stress, up-regulation of ER stress response, up-regulation of cellular response to endoplasmic reticulum stress, up-regulation of response to ER stress, up-regulation of response to endoplasmic reticulum stress, upregulation of ER stress response, upregulation of cellular response to endoplasmic reticulum stress, upregulation of response to ER stress, upregulation of response to endoplasmic reticulum stress, activation of ER stress response, activation of cellular response to endoplasmic reticulum stress, activation of response to ER stress, activation of response to endoplasmic reticulum stress References: PMID:21803450 Sources: GOC:TermGenie, GOC:aruk, GOC:bc, GO_REF:0000058 Definition: Any process that activates or increases the frequency, rate or extent of response to endoplasmic reticulum stress. Subtypes: GO:1900103, positive regulation of endoplasmic reticulum stress-induced intrinsic apoptotic signaling pathway [GO:1902237], positive regulation of ERAD pathway [GO:1904294] Relationships: is a type of positive regulation of cellular process [GO:0048522]; is a type of positive regulation of response to stimulus [GO:0048584]; is a type of regulation of response to endoplasmic reticulum stress [GO:1905897]; positively regulates response to endoplasmic reticulum stress [GO:0034976]